{
  "term_label": "Unknown molecular function",
  "term_id": "UNKNOWN:0001",
  "gene_name": "Melanoma-associated antigen C2",
  "gene_symbol": "MAGEC2",
  "gene": "UniProtKB:Q9UBF1"
}